{
  "term_id": "UNKNOWN:0002",
  "gene": "UniProtKB:Q6P2I7",
  "gene_symbol": "EBLN2",
  "term_label": "Unknown biological process",
  "gene_name": "Endogenous Bornavirus-like nucleoprotein 2"
}